{
  "term_id": "GO:0006357",
  "term_label": "regulation of transcription by RNA polymerase II",
  "gene_symbol": "TFEC",
  "gene": "UniProtKB:O14948",
  "gene_name": "Transcription factor EC"
}